CXCR3 chemokine receptor binding [GO:0048248] (molecular function) Relationships: is a type of GO:0045236 References: PMID:10556837 Sources: GOC:jid Definition: Binding to a CXCR3 chemokine receptor.